{
  "gene_name": "Protocadherin-17",
  "term_id": "GO:0007155",
  "gene": "UniProtKB:O14917",
  "gene_symbol": "PCDH17",
  "term_label": "cell adhesion"
}